left anterior basal body [GO:1902671] (cellular component) Definition: Any ciliary basal body that is part of a left anterior flagellum found in Giardia species (trophozoite stage). References: PMID:16607022, PMID:5961344 Sources: GOC:TermGenie, GOC:giardia, GO_REF:0000064, ISBN:9780124260207 Also known as: cilial basal body of left anterior cilium, cilial basal body of left anterior flagellum, ciliary basal body of left anterior cilium, ciliary basal body of left anterior flagellum, cilium basal body of left anterior cilium, cilium basal body of left anterior flagellum, left anterior flagellum ciliary basal body, microtubule basal body of left anterior cilium, microtubule basal body of left anterior flagellum Relationships: is a type of ciliary basal body [GO:0036064]; is part of left anterior flagellum [GO:0097554] Note: Note that we deem cilium and microtubule-based flagellum to be equivalent. Also note that, due to the asymmetric nature of the Giardia trophozoite, this term is defined spatially as the trophozoite is viewed from the dorsal side, with the two nuclei dorsal to the ventral disc, and the ventral disc toward the anterior.